{
  "gene_symbol": "STAR",
  "term_label": "intracellular cholesterol transport",
  "gene_name": "Steroidogenic acute regulatory protein, mitochondrial",
  "term_id": "GO:0032367",
  "gene": "UniProtKB:P49675"
}